{
  "term_label": "Unknown molecular function",
  "gene_name": "Transcription factor Dp family member 3",
  "term_id": "UNKNOWN:0001",
  "gene": "UniProtKB:Q5H9I0",
  "gene_symbol": "TFDP3"
}